{
  "gene": "UniProtKB:Q12874",
  "term_label": "spliceosomal complex",
  "gene_symbol": "SF3A3",
  "term_id": "GO:0005681",
  "gene_name": "Splicing factor 3A subunit 3"
}